acetoacetate-CoA ligase activity [GO:0030729] (molecular function) Definition: Catalysis of the reaction: acetoacetate + ATP + CoA = acetoacetyl-CoA + AMP + diphosphate + H+. Sources: EC:6.2.1.16, RHEA:16117 Also known as: acetoacetyl-CoA synthetase activity, acetoacetate:CoA ligase (AMP-forming) Relationships: is_a GO:0016405; is a type of acid-thiol ligase activity [GO:0016878]